interleukin-25 production [GO:0032629] (biological process) Sources: GOC:mah Definition: The appearance of interleukin-25 due to biosynthesis or secretion following a cellular stimulus, resulting in an increase in its intracellular or extracellular levels. Also known as: IL-25 production, IL-25 secretion, IL17E secretion, interleukin-25 anabolism, interleukin-25 biosynthesis, interleukin-25 biosynthetic process, interleukin-25 formation, interleukin-25 secretion, interleukin-25 synthesis Relationships: is a type of cytokine production [GO:0001816] Regulation: regulated by regulation of interleukin-25 production [GO:0032669]; negatively regulated by negative regulation of interleukin-25 production [GO:0032709]; positively regulated by positive regulation of interleukin-25 production [GO:0032749]